{
  "gene": "UniProtKB:Q9H4D0",
  "gene_symbol": "CLSTN2",
  "gene_name": "Calsyntenin-2",
  "term_id": "GO:0007156",
  "term_label": "homophilic cell-cell adhesion"
}